cellular response to peptidoglycan [GO:0071224] (biological process) Definition: Any process that results in a change in state or activity of a cell (in terms of movement, secretion, enzyme production, gene expression, etc.) as a result of a peptidoglycan stimulus. Peptidoglycan is a bacterial cell wall macromolecule. Relationships: is a type of response to peptidoglycan [GO:0032494]; is a type of cellular response to molecule of bacterial origin [GO:0071219]; is a type of cellular response to nitrogen compound [GO:1901699]; is a type of cellular response to oxygen-containing compound [GO:1901701] Sources: GOC:mah